{
  "gene": "UniProtKB:Q9UPR0",
  "term_label": "Unknown cellular component",
  "gene_name": "Inactive phospholipase C-like protein 2",
  "term_id": "UNKNOWN:0003",
  "gene_symbol": "PLCL2"
}